{
  "term_id": "GO:0005634",
  "gene_name": "Cyclin-dependent kinase 7",
  "gene": "UniProtKB:P50613",
  "gene_symbol": "CDK7",
  "term_label": "nucleus"
}